{
  "term_label": "cytoskeletal motor activity",
  "term_id": "GO:0003774",
  "gene_name": "Myosin light chain 3",
  "gene_symbol": "MYL3",
  "gene": "UniProtKB:P08590"
}